3'-5'-DNA exonuclease activity [GO:0008296] (molecular function) Also known as: 3'-5' exodeoxyribonuclease activity, 3'-5'-exodeoxyribonuclease activity Relationships: is a type of 3'-5' exonuclease activity [GO:0008408]; is a type of DNA exonuclease activity, producing 5'-phosphomonoesters [GO:0016895] Definition: Catalysis of the sequential cleavage of mononucleotides from a free 3' terminus of a DNA molecule. Sources: GOC:mah Subtypes: single-stranded DNA 3'-5' DNA exonuclease activity [GO:0008310], double-stranded DNA 3'-5' DNA exonuclease activity [GO:0008311]